{
  "gene_symbol": "ZNF84",
  "term_id": "UNKNOWN:0002",
  "gene": "UniProtKB:P51523",
  "gene_name": "Zinc finger protein 84",
  "term_label": "Unknown biological process"
}